pyridoxal kinase activity [GO:0008478] (molecular function) Definition: Catalysis of the reaction: ATP + pyridoxal = ADP + pyridoxal 5'-phosphate. Also known as: ATP:pyridoxal 5'-phosphotransferase activity, pyridoxal 5-phosphate-kinase activity, pyridoxal kinase (phosphorylating), pyridoxal phosphokinase activity, pyridoxamine kinase activity, pyridoxine kinase activity, vitamin B(6) kinase activity, vitamin B6 kinase activity Relationships: is a type of kinase activity [GO:0016301]; is a type of phosphotransferase activity, alcohol group as acceptor [GO:0016773] Sources: EC:2.7.1.35